{
  "term_id": "GO:0043083",
  "term_label": "synaptic cleft",
  "gene_symbol": "CBLN1",
  "gene_name": "Cerebellin-1",
  "gene": "UniProtKB:P23435"
}